{
  "gene_name": "Ankyrin repeat domain-containing protein 12",
  "gene_symbol": "ANKRD12",
  "term_label": "Unknown molecular function",
  "gene": "UniProtKB:Q6UB98",
  "term_id": "UNKNOWN:0001"
}